nuclear cortical migration [GO:0035192] (biological process) Relationships: is a type of syncytial nuclear migration [GO:0035190] Definition: The symmetric outward movement of the syncytial nuclei from their positions in the ellipsoid toward the periphery of the embryo, during mitotic cycles 8 and 9. This movement results in the placement of nuclei in a uniform monolayer at the cortex of the developing embryo. References: PMID:8314839